{
  "term_label": "RNA polymerase II cis-regulatory region sequence-specific DNA binding",
  "term_id": "GO:0000978",
  "gene_symbol": "ZNF317",
  "gene_name": "Zinc finger protein 317",
  "gene": "UniProtKB:Q96PQ6"
}